homeostatic process [GO:0042592] (biological process) Also known as: homeostasis, activation of homeostatic process, inhibition of homeostatic process, negative regulation of homeostatic process, positive regulation of homeostatic process, regulation of homeostatic process Subtypes: cellular homeostasis [GO:0019725], multicellular organismal-level homeostasis [GO:0048871], chemical homeostasis [GO:0048878] Sources: GOC:jl, ISBN:0395825172 Definition: Any biological process involved in the maintenance of an internal steady state. Relationships: is a type of biological_process [GO:0008150]